positive regulation of metanephric glomerulus development [GO:0072300] (biological process) Sources: GOC:mtg_kidney_jan10 Relationships: is a type of GO:0072216; is_a regulation of metanephric glomerulus development [GO:0072298]; is_a positive regulation of glomerulus development [GO:0090193]; RO_0002213 metanephric glomerulus development [GO:0072224] Definition: Any process that increases the rate, frequency or extent of metanephric glomerulus development, the progression of the metanephric glomerulus over time from its initial formation until its mature state. The metanephric glomerulus is a capillary tuft surrounded by Bowman's capsule in nephrons of the vertebrate kidney, or metanephros.